{
  "gene": "UniProtKB:Q9NUT2",
  "term_id": "GO:0055085",
  "term_label": "transmembrane transport",
  "gene_symbol": "ABCB8",
  "gene_name": "Mitochondrial potassium channel ATP-binding subunit"
}